{
  "term_id": "UNKNOWN:0003",
  "gene_symbol": "C9orf131",
  "gene_name": "Uncharacterized protein C9orf131",
  "gene": "UniProtKB:Q5VYM1",
  "term_label": "Unknown cellular component"
}